{
  "gene_symbol": "ZNF35",
  "gene": "UniProtKB:P13682",
  "term_label": "nucleus",
  "term_id": "GO:0005634",
  "gene_name": "Zinc finger protein 35"
}